cartilage homeostasis [GO:1990079] (biological process) Definition: A tissue homeostatic process involved in the maintenance of an internal equilibrium within cartilage, including control of cellular proliferation and death and control of metabolic function. References: PMID:21652695 Sources: GOC:hjd Relationships: is_a tissue homeostasis [GO:0001894] Also known as: negative regulation of cartilage homeostasis, positive regulation of cartilage homeostasis, regulation of cartilage homeostasis